{
  "term_label": "regulation of immune system process",
  "gene_name": "Prolactin-inducible protein",
  "gene_symbol": "PIP",
  "gene": "UniProtKB:P12273",
  "term_id": "GO:0002682"
}